{
  "term_id": "GO:0016925",
  "gene_name": "E3 ubiquitin-protein ligase Topors",
  "gene_symbol": "TOPORS",
  "gene": "UniProtKB:Q9NS56",
  "term_label": "protein sumoylation"
}